positive regulation of pseudohyphal septin ring assembly [GO:0062165] (BP) Relationships: is a type of GO:0031334; is a type of positive regulation of cytoskeleton organization [GO:0051495]; is a type of regulation of pseudohyphal septin ring assembly [GO:0062164]; is_a GO:1902117; positively regulates pseudohyphal septin ring assembly [GO:0062163] References: PMID:29567712 Definition: Any process that increases the rate, frequency or extent of pseudohyphal septin ring formation.